{
  "gene_name": "PTTG1IP family member 2",
  "gene_symbol": "PTTG1IP2",
  "term_id": "UNKNOWN:0003",
  "term_label": "Unknown cellular component",
  "gene": "UniProtKB:P0DTF9"
}